venom-mediated paralysis [GO:0044616] (biological process) References: PMID:28422078, PMID:36668869 Definition: A process in which an organism induces paralysis in another organism via the action of a venom. Paralysis is the loss of the ability to voluntarily control muscles. This can occur by blocking nerve signals at the neuromuscular junction or by directly interfering with muscle contraction. Also known as: envenomation resulting in paralysis in another organism, modulation of relaxation of muscle in other organism, regulation of relaxation of muscle in other organism, modulation of relaxation of muscle in another organism Relationships: is a type of venom-mediated perturbation of nervous system process [GO:0140136]